{
  "gene_symbol": "VPS50",
  "term_id": "GO:1990745",
  "term_label": "EARP complex",
  "gene": "UniProtKB:Q96JG6",
  "gene_name": "Syndetin"
}